{
  "gene_name": "E3 ubiquitin-protein ligase HACE1",
  "gene": "UniProtKB:Q8IYU2",
  "term_id": "GO:0006511",
  "gene_symbol": "HACE1",
  "term_label": "ubiquitin-dependent protein catabolic process"
}